{
  "gene_symbol": "IRF8",
  "term_label": "DNA-binding transcription factor activity, RNA polymerase II-specific",
  "term_id": "GO:0000981",
  "gene_name": "Interferon regulatory factor 8",
  "gene": "UniProtKB:Q02556"
}